{
  "gene_name": "Semaphorin-3B",
  "gene": "UniProtKB:Q13214",
  "term_label": "semaphorin receptor binding",
  "term_id": "GO:0030215",
  "gene_symbol": "SEMA3B"
}